pseudouridine synthase activity [GO:0009982] (molecular function) Definition: Catalysis of the reaction: a uridine in RNA = a pseudouridine in RNA. Conversion of uridine in an RNA molecule to pseudouridine by rotation of the C1'-N-1 glycosidic bond of uridine in RNA to a C1'-C5. Relationships: is a type of GO:0016866 Subtypes: tRNA pseudouridine synthase activity [GO:0106029], GO:0106032, rRNA pseudouridine synthase activity [GO:0120159] Sources: GOC:mah, RHEA:48348 Note: Note that this term should not be confused with 'pseudouridylate synthase activity ; GO:0004730', which refers to the formation of free pseudouridine from uracil and ribose-5-phosphate.